{
  "gene_name": "Ral GTPase-activating protein subunit alpha-2",
  "term_label": "GTPase activator activity",
  "term_id": "GO:0005096",
  "gene_symbol": "RALGAPA2",
  "gene": "UniProtKB:Q2PPJ7"
}